{
  "gene_symbol": "NDUFB11",
  "term_id": "UNKNOWN:0002",
  "term_label": "Unknown biological process",
  "gene_name": "NADH dehydrogenase [ubiquinone] 1 beta subcomplex subunit 11, mitochondrial",
  "gene": "UniProtKB:Q9NX14"
}